neurotransmitter secretion involved in regulation of skeletal muscle contraction [GO:0014860] (biological process) Relationships: is a type of neurotransmitter secretion [GO:0007269]; is part of regulation of skeletal muscle contraction by neural stimulation via neuromuscular junction [GO:0014852] Also known as: neurotransmitter secretion involved in control of skeletal muscle contraction Sources: GOC:dph, GOC:mtg_muscle, GOC:tb Definition: The regulated release of neurotransmitter into the synaptic cleft involved in skeletal muscle contraction. A neurotransmitter is any of a group of substances that are released on excitation from the axon terminal of a presynaptic neuron of the central or peripheral nervous system and travel across the synaptic cleft to either excite or inhibit the target cell. Among the many substances that have the properties of a neurotransmitter are acetylcholine, noradrenaline, adrenaline, dopamine, glycine, gamma aminobutyrate, glutamic acid, substance P, enkephalins, endorphins and serotonin.